{
  "gene_name": "Microtubule-associated protein RP_EB family member 2",
  "gene_symbol": "MAPRE2",
  "gene": "UniProtKB:Q15555",
  "term_label": "spindle midzone",
  "term_id": "GO:0051233"
}